{
  "gene": "UniProtKB:Q9UPX8",
  "term_id": "GO:0043197",
  "term_label": "dendritic spine",
  "gene_name": "SH3 and multiple ankyrin repeat domains protein 2",
  "gene_symbol": "SHANK2"
}